diorcinol catabolic process [GO:1900571] (BP) Sources: GOC:TermGenie, GOC:di Also known as: diorcinol breakdown, diorcinol catabolism, diorcinol degradation Relationships: is a type of phenol-containing compound catabolic process [GO:0019336]; is a type of secondary metabolite catabolic process [GO:0090487]; is a type of diorcinol metabolic process [GO:1900570]; is a type of ether catabolic process [GO:1901502] Definition: The chemical reactions and pathways resulting in the breakdown of diorcinol.